{
  "term_id": "GO:0007339",
  "gene_symbol": "ZP2",
  "term_label": "binding of sperm to zona pellucida",
  "gene": "UniProtKB:Q05996",
  "gene_name": "Zona pellucida sperm-binding protein 2"
}